translocon complex [GO:0071256] (cellular component) Definition: A protein complex that constitutes a specific site of protein translocation across the endoplasmic reticulum, which involves the signal recognition particle receptor. The complex contains a core heterotrimer of alpha, beta and gamma subunits, and may contain additional proteins. References: PMID:10611978, PMID:18166647, PMID:8612571 Sources: GOC:mah Subtypes: Sec61 translocon complex [GO:0005784], Ssh1 translocon complex [GO:0071261] Relationships: is_a membrane protein complex [GO:0098796]; is_a endoplasmic reticulum protein-containing complex [GO:0140534]; is part of rough endoplasmic reticulum membrane [GO:0030867] Also known as: Sec complex-associated translocon complex